{
  "term_id": "GO:0000978",
  "gene": "UniProtKB:Q9Y692",
  "gene_symbol": "GMEB1",
  "term_label": "RNA polymerase II cis-regulatory region sequence-specific DNA binding",
  "gene_name": "Glucocorticoid modulatory element-binding protein 1"
}